{
  "gene": "UniProtKB:Q9Y3D9",
  "gene_name": "Small ribosomal subunit protein mS23",
  "gene_symbol": "MRPS23",
  "term_label": "mitochondrion",
  "term_id": "GO:0005739"
}